{
  "gene_symbol": "NCBP2AS2",
  "term_label": "Unknown cellular component",
  "gene": "UniProtKB:Q69YL0",
  "term_id": "UNKNOWN:0003",
  "gene_name": "Protein NCBP2AS2"
}